{
  "term_id": "GO:0001886",
  "gene": "UniProtKB:P39060",
  "gene_name": "Collagen alpha-1(XVIII) chain",
  "term_label": "endothelial cell morphogenesis",
  "gene_symbol": "COL18A1"
}